part of [BFO:0000050] (external) Relationships: inverseOf has part [BFO:0000051]